{
  "term_label": "innate immune response",
  "gene_name": "Beta-defensin 135",
  "term_id": "GO:0045087",
  "gene": "UniProtKB:Q30KP9",
  "gene_symbol": "DEFB135"
}